nucleotide-excision repair, DNA damage recognition [GO:0000715] (biological process) Also known as: pyrimidine-dimer repair, DNA damage recognition Relationships: is_a GO:0051276; is part of nucleotide-excision repair [GO:0006289] Subtypes: transcription-coupled nucleotide-excision repair, DNA damage recognition [GO:0000716] Definition: The identification of lesions in DNA, such as pyrimidine-dimers, intrastrand cross-links, and bulky adducts. The wide range of substrate specificity suggests the repair complex recognizes distortions in the DNA helix. References: PMID:10197977 Sources: GOC:elh